{
  "gene": "UniProtKB:Q9Y3R0",
  "term_id": "UNKNOWN:0003",
  "gene_symbol": "GRIP1",
  "gene_name": "Glutamate receptor-interacting protein 1",
  "term_label": "Unknown cellular component"
}